{
  "term_label": "unfolded protein binding",
  "gene_name": "DnaJ homolog subfamily B member 7",
  "term_id": "GO:0051082",
  "gene": "UniProtKB:Q7Z6W7",
  "gene_symbol": "DNAJB7"
}